luteinizing hormone signaling pathway involved in ovarian follicle development [GO:0035471] (biological process) Definition: The series of molecular signals initiated by luteinizing hormone binding to a receptor, where the activated receptor signals via downstream effectors that contribute to progression of the ovarian follicle over time, from its formation to the mature structure. Also known as: luteinizing hormone signalling pathway involved in ovarian follicle development Sources: GOC:bf Relationships: is a type of GO:0042700; is part of ovarian follicle development [GO:0001541]